{
  "gene": "UniProtKB:Q8WZ94",
  "gene_symbol": "OR5P3",
  "term_id": "GO:0004984",
  "term_label": "olfactory receptor activity",
  "gene_name": "Olfactory receptor 5P3"
}